regulation of xanthophore differentiation [GO:0050938] (biological process) Definition: Any process that modulates the frequency, rate or extent of xanthophore differentiation. Note: Note that this term refers to xanthophores in the sense of specialized pigment-producing cells, and should not be confused with the cellular component term 'xanthophore ; GO:0031633', which refers to a subcellular structure. Relationships: is a type of regulation of pigment cell differentiation [GO:0050932]; regulates xanthophore differentiation [GO:0050936] Subtypes: GO:0050944, positive regulation of xanthophore differentiation [GO:0050946] Sources: GOC:ai